{
  "gene_name": "HLA class I histocompatibility antigen, alpha chain E",
  "term_id": "GO:0006955",
  "term_label": "immune response",
  "gene": "UniProtKB:P13747",
  "gene_symbol": "HLA-E"
}